{
  "gene_symbol": "DNMT1",
  "gene_name": "DNA (cytosine-5)-methyltransferase 1",
  "gene": "UniProtKB:P26358",
  "term_id": "GO:0003677",
  "term_label": "DNA binding"
}